{
  "term_label": "plasma membrane",
  "gene_symbol": "AVPR1A",
  "term_id": "GO:0005886",
  "gene": "UniProtKB:P37288",
  "gene_name": "Vasopressin V1a receptor"
}